lipoate-protein ligase activity [GO:0016979] (molecular function) Relationships: is a type of GO:0016779; is a type of ligase activity, forming carbon-nitrogen bonds [GO:0016879]; is_a catalytic activity, acting on a protein [GO:0140096] Definition: Catalysis of the lipoylation of a protein in two steps: ATP + (R)-lipoate + a [lipoyl-carrier protein]-L-lysine = a [lipoyl-carrier protein]-N6-(lipoyl)lysine + AMP + diphosphate (overall reaction): (1) ATP + (R)-lipoate = lipoyl-AMP + diphosphate; (2) lipoyl-AMP + a [lipoyl-carrier protein]-L-lysine = a [lipoyl-carrier protein]-N6-(lipoyl)lysine + AMP. References: PMID:16141198, PMID:17570395 Sources: RHEA:49288 Also known as: lipoate-protein ligase A activity, lipoate-protein ligase B activity, lipoate-protein ligase activity (lipoylation of glycine cleavage complex)